{
  "gene_name": "Microtubule-associated proteins 1A_1B light chain 3A",
  "term_id": "GO:0097352",
  "term_label": "autophagosome maturation",
  "gene": "UniProtKB:Q9H492",
  "gene_symbol": "MAP1LC3A"
}